{
  "term_label": "Unknown cellular component",
  "gene": "UniProtKB:Q13145",
  "gene_symbol": "BAMBI",
  "term_id": "UNKNOWN:0003",
  "gene_name": "BMP and activin membrane-bound inhibitor homolog"
}